{
  "gene_symbol": "TP73",
  "term_label": "regulation of apoptotic process",
  "gene": "UniProtKB:O15350",
  "term_id": "GO:0042981",
  "gene_name": "Tumor protein p73"
}